{
  "gene": "UniProtKB:Q14511",
  "term_label": "cell surface receptor protein tyrosine kinase signaling pathway",
  "gene_name": "Enhancer of filamentation 1",
  "gene_symbol": "NEDD9",
  "term_id": "GO:0007169"
}